{
  "gene": "UniProtKB:O00194",
  "gene_symbol": "RAB27B",
  "term_id": "GO:0003924",
  "term_label": "GTPase activity",
  "gene_name": "Ras-related protein Rab-27B"
}